{
  "gene_symbol": "SLC39A8",
  "gene": "UniProtKB:Q9C0K1",
  "term_id": "GO:0005385",
  "term_label": "zinc ion transmembrane transporter activity",
  "gene_name": "Metal cation symporter ZIP8"
}